{
  "term_label": "nucleus",
  "gene": "UniProtKB:Q9UJC5",
  "term_id": "GO:0005634",
  "gene_name": "SH3 domain-binding glutamic acid-rich-like protein 2",
  "gene_symbol": "SH3BGRL2"
}